5-exo-hydroxycamphor dehydrogenase activity [GO:0018452] (MF) Definition: Catalysis of the reaction: 5-exo-hydroxycamphor + NAD+ = NADH + H+ + 2,5-diketocamphane. Sources: UM-BBD_reactionID:r0427 Relationships: is a type of oxidoreductase activity, acting on the CH-OH group of donors, NAD or NADP as acceptor [GO:0016616]